{
  "term_label": "calcium ion binding",
  "gene_symbol": "S100A2",
  "gene": "UniProtKB:P29034",
  "gene_name": "Protein S100-A2",
  "term_id": "GO:0005509"
}